galactose oxidase activity [GO:0045480] (molecular function) Sources: EC:1.1.3.9 Definition: Catalysis of the reaction: D-galactose + O2 = D-galacto-hexodialdose + hydrogen peroxide. Relationships: is a type of oxidoreductase activity, acting on the CH-OH group of donors, oxygen as acceptor [GO:0016899] Also known as: D-galactose oxidase activity, D-galactose:oxygen 6-oxidoreductase activity, beta-galactose oxidase activity